nucleoside bisphosphate biosynthetic process [GO:0033866] (biological process) Relationships: is a type of GO:0033865; is a type of GO:1901293 Sources: GOC:mah, GOC:pde Subtypes: ribonucleoside bisphosphate biosynthetic process [GO:0034030], GO:0034033 Also known as: nucleoside bisphosphate anabolism, nucleoside bisphosphate biosynthesis, nucleoside bisphosphate formation, nucleoside bisphosphatehate synthesis Definition: The chemical reactions and pathways resulting in the formation of a nucleoside bisphosphate, a compound consisting of a nucleobase linked to a deoxyribose or ribose sugar esterified with one phosphate group attached to each of two different hydroxyl groups on the sugar.